{
  "term_label": "RNA polymerase II preinitiation complex assembly",
  "gene_symbol": "TAF11L3",
  "gene": "UniProtKB:A0A1W2PRV1",
  "gene_name": "TATA-box-binding protein-associated factor 11-like protein 3",
  "term_id": "GO:0051123"
}